{
  "gene_symbol": "CEP126",
  "gene": "UniProtKB:Q9P2H0",
  "term_id": "GO:0031122",
  "gene_name": "Centrosomal protein of 126 kDa",
  "term_label": "cytoplasmic microtubule organization"
}